{
  "term_id": "UNKNOWN:0003",
  "gene": "UniProtKB:Q7L2K0",
  "gene_symbol": "TEDC2",
  "gene_name": "Tubulin epsilon and delta complex protein 2",
  "term_label": "Unknown cellular component"
}